protein-arginine deiminase activity [GO:0004668] (molecular function) Definition: Catalysis of the reaction: H2O + L-arginyl-[protein] = L-citrullyl-[protein] + NH4+, resulting in citrullination of the target protein. This reaction is calcium-dependent. References: PMID:27393304 Also known as: peptidylarginine deiminase activity, protein-L-arginine iminohydrolase activity Relationships: is a type of hydrolase activity, acting on carbon-nitrogen (but not peptide) bonds, in linear amidines [GO:0016813] Subtypes: histone arginine deiminase activity [GO:0140794]